smoothened signaling pathway involved in lung development [GO:0060506] (biological process) Sources: GOC:dph, GOC:mtg_lung Definition: The series of molecular signals generated as a consequence of activation of the transmembrane Smoothened-type protein. This process contributes to lung development. Also known as: hedgehog signaling pathway involved in lung development, hh signaling pathway involved in lung development, smoothened signalling pathway involved in lung development Relationships: is a type of smoothened signaling pathway [GO:0007224]; is part of GO:0060495